{
  "gene_name": "X antigen family member 3",
  "term_label": "Unknown biological process",
  "gene_symbol": "XAGE3",
  "gene": "UniProtKB:Q8WTP9",
  "term_id": "UNKNOWN:0002"
}